{
  "gene_name": "Paired mesoderm homeobox protein 2A",
  "gene": "UniProtKB:O14813",
  "term_id": "GO:0000977",
  "term_label": "RNA polymerase II transcription regulatory region sequence-specific DNA binding",
  "gene_symbol": "PHOX2A"
}